{
  "term_id": "GO:0006412",
  "gene_name": "Small ribosomal subunit protein eS1",
  "gene_symbol": "RPS3A",
  "gene": "UniProtKB:P61247",
  "term_label": "translation"
}